regulation of pancreatic A cell differentiation [GO:2000226] (biological process) Sources: GOC:mah Also known as: regulation of pancreatic alpha cell differentiation Definition: Any process that modulates the frequency, rate or extent of pancreatic A cell differentiation. Relationships: is a type of regulation of epithelial cell differentiation [GO:0030856]; regulates pancreatic A cell differentiation [GO:0003310] Subtypes: GO:2000227, positive regulation of pancreatic A cell differentiation [GO:2000228]